glyoxylate metabolic process [GO:0046487] (biological process) Subtypes: glyoxylate cycle [GO:0006097], glyoxylate catabolic process [GO:0009436] Sources: ISBN:0198506732 Definition: The chemical reactions and pathways involving glyoxylate, the anion of glyoxylic acid, HOC-COOH. Also known as: glyoxylate metabolism Relationships: is a type of aldehyde metabolic process [GO:0006081]; is a type of monocarboxylic acid metabolic process [GO:0032787]